{
  "gene": "UniProtKB:Q96HJ9",
  "term_label": "Unknown biological process",
  "term_id": "UNKNOWN:0002",
  "gene_name": "Protein FMC1 homolog",
  "gene_symbol": "FMC1"
}